{
  "gene_name": "Protein TASOR 2",
  "term_label": "Unknown molecular function",
  "gene": "UniProtKB:Q5VWN6",
  "gene_symbol": "TASOR2",
  "term_id": "UNKNOWN:0001"
}